cytokine production [GO:0001816] (biological process) Also known as: cytokine biosynthetic process, cytokine metabolic process, cytokine secretion, interferon production, interferon secretion, interleukin production, interleukin secretion Sources: GOC:add, ISBN:0781735149 Note: Note that this term is in the subset of terms that should not be used for direct gene product annotation. Instead, select one of the 'regulation' children terms. Regulation: regulated by regulation of cytokine production [GO:0001817]; negatively regulated by negative regulation of cytokine production [GO:0001818]; RO_0002213 by GO:0001819 Relationships: is a type of gene expression [GO:0010467]; is a type of multicellular organismal process [GO:0032501] Subtypes: cytokine production involved in immune response [GO:0002367], cytokine production involved in inflammatory response [GO:0002534], vascular endothelial growth factor production [GO:0010573], GO:0032601, chemokine production [GO:0032602], GO:0032604, GO:0032605, type I interferon production [GO:0032606], type II interferon production [GO:0032609], interleukin-1 production [GO:0032612], interleukin-10 production [GO:0032613], interleukin-11 production [GO:0032614], GO:0032615, interleukin-13 production [GO:0032616], interleukin-15 production [GO:0032618], interleukin-16 production [GO:0032619], interleukin-17 production [GO:0032620], interleukin-18 production [GO:0032621], interleukin-19 production [GO:0032622], GO:0032623, interleukin-20 production [GO:0032624], interleukin-21 production [GO:0032625], interleukin-22 production [GO:0032626], interleukin-23 production [GO:0032627], interleukin-24 production [GO:0032628], interleukin-25 production [GO:0032629], interleukin-26 production [GO:0032630], GO:0032631, GO:0032632, interleukin-4 production [GO:0032633], GO:0032634, GO:0032635, interleukin-7 production [GO:0032636], interleukin-8 production [GO:0032637], interleukin-9 production [GO:0032638], type III interferon production [GO:0034343], macrophage colony-stimulating factor production [GO:0036301], GO:0044467, macrophage migration inhibitory factor production [GO:0044807], GO:0044808, GO:0070753, GO:0071604, granulocyte colony-stimulating factor production [GO:0071611], GO:0071706, interleukin-30 production [GO:0072633], interleukin-31 production [GO:0072635], interleukin-32 production [GO:0072637], interleukin-33 production [GO:0072639], GO:0090269, platelet-derived growth factor production [GO:0090360], amphiregulin production [GO:0140730], XCL1 production [GO:0140779], interleukin-37 production [GO:0150137], GO:0150155, endothelin production [GO:1990775] Definition: The appearance of a cytokine due to biosynthesis or secretion following a cellular stimulus, resulting in an increase in its intracellular or extracellular levels.